regulation of epithelial tube formation [GO:1905276] (biological process) Definition: Any process that modulates the frequency, rate or extent of epithelial tube formation. Relationships: is a type of regulation of morphogenesis of an epithelium [GO:1905330]; is a type of GO:2000026; regulates GO:0072175 Note: An example of this is MMRN2 in human (Q9H8L6) in PMID:25745997 (inferred from direct assay). Subtypes: regulation of ureteric bud formation [GO:0072106], negative regulation of epithelial tube formation [GO:1905277], positive regulation of epithelial tube formation [GO:1905278] References: PMID:25745997 Sources: GOC:TermGenie, GOC:bhm, GO_REF:0000058